{
  "gene_symbol": "NRF1",
  "term_id": "GO:0000978",
  "gene": "UniProtKB:Q16656",
  "term_label": "RNA polymerase II cis-regulatory region sequence-specific DNA binding",
  "gene_name": "Nuclear respiratory factor 1"
}